social behavior [GO:0035176] (biological process) Definition: Behavior directed towards society, or taking place between members of the same species. Occurs predominantly, or only, in individuals that are part of a group. Subtypes: GO:0160306 Relationships: is a type of behavior [GO:0007610]; is a type of biological process involved in intraspecies interaction between organisms [GO:0051703] Note: Behavior such as predation which involves members of different species is not social. Communication between members of different species is also not social behavior. References: PMID:12848939 Sources: GOC:jh2, Wikipedia:Social_behavior Also known as: social behaviour, cooperative behavior